{
  "gene_name": "Synaptotagmin-15B",
  "term_label": "calcium ion sensor activity",
  "gene_symbol": "SYT15B",
  "term_id": "GO:0061891",
  "gene": "UniProtKB:X6R8R1"
}